{
  "gene_name": "Max-binding protein MNT",
  "term_label": "DNA-binding transcription factor activity, RNA polymerase II-specific",
  "gene_symbol": "MNT",
  "term_id": "GO:0000981",
  "gene": "UniProtKB:Q99583"
}